photoreceptor ribbon synapse [GO:0098684] (cellular component) Definition: A ribbon synapse between a retinal photoreceptor cell (rod or cone) and a retinal bipolar cell. These contain a plate-like synaptic ribbon. References: PMID:15626493 Relationships: is a type of ribbon synapse [GO:0097470]